nocardicin-A epimerase activity [GO:0050143] (molecular function) Relationships: is a type of racemase and epimerase activity, acting on amino acids and derivatives [GO:0016855] Definition: Catalysis of the reaction: isonocardicin A = nocardicin A. May also catalyse the epimerisation of isonocardicin C, but the in vivo substrate appears to be isonocardicin A. Sources: EC:5.1.1.14, RHEA:22792 Also known as: isonocardicin A epimerase activity